negative regulation of convergent extension involved in neural plate elongation [GO:1904131] (BP) Relationships: is a type of GO:1904104; is a type of regulation of convergent extension involved in neural plate elongation [GO:1904130]; negatively regulates convergent extension involved in neural plate elongation [GO:0022007] References: PMID:24892953 Sources: GOC:TermGenie, GOC:dph, GO_REF:0000058 Definition: Any process that stops, prevents or reduces the frequency, rate or extent of convergent extension involved in neural plate elongation. Also known as: down regulation of convergent extension involved in neural plate elongation, down-regulation of convergent extension involved in neural plate elongation, downregulation of convergent extension involved in neural plate elongation, inhibition of convergent extension involved in neural plate elongation